{
  "gene_name": "NGFI-A-binding protein 1",
  "term_id": "GO:0005634",
  "term_label": "nucleus",
  "gene_symbol": "NAB1",
  "gene": "UniProtKB:Q13506"
}